{
  "gene": "UniProtKB:P62079",
  "term_label": "plasma membrane",
  "gene_name": "Tetraspanin-5",
  "gene_symbol": "TSPAN5",
  "term_id": "GO:0005886"
}